D-alanyl carrier activity [GO:0036370] (molecular function) Also known as: D-alanyl carrier protein Definition: Binding a D-alanine and presenting it for processing or offloading to a cognate enzyme. Covalently binds the D-alanine via a phosphopantetheine prosthetic group and mediates protein-protein interactions with the enzyme conferring specificity. The carrier protein provides an essential link between the D-alanine-D-alanyl carrier protein ligase and the incorporation of D-alanine into lipoteichoic acid by transferring activated D-alanine to cell membrane phosphatidylglycerol (PG). References: PMID:11222605, PMID:22750871, PMID:8682792 Sources: GOC:crds Relationships: is a type of phosphopantetheine-dependent carrier activity [GO:0140414]; is part of teichoic acid D-alanylation [GO:0070400]